skeletal muscle satellite stem cell asymmetric division [GO:0014833] (biological process) Also known as: satellite cell asymmetric division Relationships: is a type of somatic stem cell division [GO:0048103]; is a type of asymmetric stem cell division [GO:0098722]; is part of skeletal muscle tissue development [GO:0007519] References: PMID:16607119 Sources: GOC:ef, GOC:mtg_muscle Subtypes: GO:0014716 Definition: The asymmetric division of a skeletal muscle satellite stem cell to produce two daughter cells, one of which is destined to differentiate and the other to be a quiescent cell that restocks the satellite cell pool.